{
  "gene": "UniProtKB:Q6ZQW0",
  "term_label": "cytoplasm",
  "gene_symbol": "IDO2",
  "term_id": "GO:0005737",
  "gene_name": "Indoleamine 2,3-dioxygenase 2"
}